{
  "term_label": "amyloid-beta clearance by cellular catabolic process",
  "gene": "UniProtKB:P16671",
  "gene_name": "Platelet glycoprotein 4",
  "gene_symbol": "CD36",
  "term_id": "GO:0150094"
}